{
  "term_id": "GO:0005634",
  "term_label": "nucleus",
  "gene_symbol": "VEZF1",
  "gene_name": "Vascular endothelial zinc finger 1",
  "gene": "UniProtKB:Q14119"
}